{
  "term_label": "granulocyte colony-stimulating factor receptor binding",
  "gene_name": "Granulocyte colony-stimulating factor",
  "term_id": "GO:0005130",
  "gene_symbol": "CSF3",
  "gene": "UniProtKB:P09919"
}